{
  "gene_name": "Olfactory receptor 6C74",
  "term_label": "olfactory receptor activity",
  "gene_symbol": "OR6C74",
  "gene": "UniProtKB:A6NCV1",
  "term_id": "GO:0004984"
}